{
  "term_label": "neuropeptide signaling pathway",
  "term_id": "GO:0007218",
  "gene_symbol": "NPPB",
  "gene_name": "Natriuretic peptides B",
  "gene": "UniProtKB:P16860"
}